{
  "gene": "UniProtKB:Q8NGF7",
  "gene_symbol": "OR5B17",
  "term_label": "Unknown cellular component",
  "term_id": "UNKNOWN:0003",
  "gene_name": "Olfactory receptor 5B17"
}